{
  "gene_symbol": "TFIP11",
  "gene": "UniProtKB:Q9UBB9",
  "gene_name": "Tuftelin-interacting protein 11",
  "term_label": "Unknown molecular function",
  "term_id": "UNKNOWN:0001"
}